{
  "gene_symbol": "OR4C16",
  "term_label": "olfactory receptor activity",
  "gene": "UniProtKB:Q8NGL9",
  "term_id": "GO:0004984",
  "gene_name": "Olfactory receptor 4C16"
}